{
  "term_id": "GO:0033063",
  "gene": "UniProtKB:O75771",
  "gene_name": "DNA repair protein RAD51 homolog 4",
  "gene_symbol": "RAD51D",
  "term_label": "Rad51B-Rad51C-Rad51D-XRCC2 complex"
}